{
  "term_label": "fibroblast growth factor receptor binding",
  "term_id": "GO:0005104",
  "gene": "UniProtKB:P09038",
  "gene_symbol": "FGF2",
  "gene_name": "Fibroblast growth factor 2"
}